{
  "gene_symbol": "RFC1",
  "term_id": "UNKNOWN:0002",
  "term_label": "Unknown biological process",
  "gene_name": "Replication factor C subunit 1",
  "gene": "UniProtKB:P35251"
}